sucrose-phosphate phosphatase activity [GO:0050307] (molecular function) Relationships: is a type of sugar-phosphatase activity [GO:0050308] Also known as: sucrose-6F-phosphate phosphohydrolase activity, sucrose-phosphate phosphohydrolase activity Definition: Catalysis of the reaction: sucrose 6F-phosphate + H2O = sucrose + phosphate. Sources: EC:3.1.3.24, MetaCyc:SUCROSE-PHOSPHATASE-RXN